{
  "gene_symbol": "CADM2",
  "gene_name": "Cell adhesion molecule 2",
  "term_id": "UNKNOWN:0001",
  "gene": "UniProtKB:Q8N3J6",
  "term_label": "Unknown molecular function"
}